Gram-negative-bacterium-type cell wall biogenesis [GO:0043164] (biological process) Relationships: is a type of peptidoglycan-based cell wall biogenesis [GO:0009273] Also known as: cell wall anabolism, cell wall assembly, cell wall biosynthetic process, cell wall formation, cell wall synthesis, 1-2nm peptidoglycan-based cell wall biogenesis Definition: A cellular process that results in the biosynthesis of constituent macromolecules, assembly, and arrangement of constituent parts of a cell wall of the type found in Gram-negative bacteria. The cell wall is the rigid or semi-rigid envelope lying outside the cell membrane. Sources: GOC:jl, GOC:mtg_sensu, ISBN:0815108893